regulation of cellular response to alkaline pH [GO:1900067] (biological process) Subtypes: negative regulation of cellular response to alkaline pH [GO:1900068] Relationships: is a type of regulation of response to stimulus [GO:0048583]; is a type of regulation of cellular process [GO:0050794]; regulates cellular response to alkaline pH [GO:0071469] Definition: Any process that modulates the frequency, rate or extent of cellular response to alkalinity. Also known as: regulation of cellular response to alkalinity, regulation of cellular response to basic pH References: PMID:12509465, PMID:17023428 Sources: GOC:TermGenie, GOC:dgf